glial filament [GO:0097426] (cellular component) Relationships: is a type of intermediate filament [GO:0005882] Sources: NIF_Subcellular:sao1863852493 Definition: An intermediate filament composed of glial fibrillary acidic protein (GFAP) and found in astrocytes.